{
  "gene_symbol": "UGT1A3",
  "gene": "UniProtKB:P35503",
  "term_id": "GO:0004857",
  "gene_name": "UDP-glucuronosyltransferase 1A3",
  "term_label": "enzyme inhibitor activity"
}